{
  "gene_symbol": "SLC26A9",
  "term_label": "sulfate transmembrane transporter activity",
  "term_id": "GO:0015116",
  "gene_name": "Solute carrier family 26 member 9",
  "gene": "UniProtKB:Q7LBE3"
}